malate import across plasma membrane [GO:0098714] (BP) Definition: The directed movement of malate from outside of a cell, across the plasma membrane and into the cytosol. Also known as: malate import into cell Sources: GOC:dos Relationships: is a type of malate transmembrane transport [GO:0071423]; is a type of import across plasma membrane [GO:0098739]